formate dehydrogenase (cytochrome-c-553) activity [GO:0047111] (molecular function) Sources: EC:1.17.2.3, MetaCyc:1.2.2.3-RXN Also known as: formate dehydrogenase (cytochrome c-553), formate:ferricytochrome-c-553 oxidoreductase activity Definition: Catalysis of the reaction: ferricytochrome C-553 + formate = ferrocytochrome C-553 + CO2. Relationships: is a type of oxidoreductase activity, acting on the aldehyde or oxo group of donors, cytochrome as acceptor [GO:0016622]